{
  "term_id": "UNKNOWN:0002",
  "gene": "UniProtKB:O00264",
  "gene_name": "Membrane-associated progesterone receptor component 1",
  "term_label": "Unknown biological process",
  "gene_symbol": "PGRMC1"
}